trichoblast maturation [GO:0048764] (biological process) Sources: GOC:jid Subtypes: root hair cell differentiation [GO:0048765] Relationships: is a type of GO:0048469; is part of trichoblast differentiation [GO:0010054] Definition: A developmental process, independent of morphogenetic (shape) change, that is required for a trichoblast cell to attain its fully functional state.